{
  "gene": "UniProtKB:Q9C0B7",
  "term_id": "UNKNOWN:0001",
  "gene_name": "Transport and Golgi organization protein 6 homolog",
  "gene_symbol": "TANGO6",
  "term_label": "Unknown molecular function"
}